{
  "gene": "UniProtKB:P35499",
  "gene_symbol": "SCN4A",
  "gene_name": "Sodium channel protein type 4 subunit alpha",
  "term_label": "cardiac muscle cell action potential involved in contraction",
  "term_id": "GO:0086002"
}